{
  "gene_name": "Thyroglobulin",
  "gene": "UniProtKB:P01266",
  "term_id": "GO:0005615",
  "gene_symbol": "TG",
  "term_label": "extracellular space"
}